{
  "term_label": "extracellular matrix organization",
  "gene_symbol": "ADAMTS19",
  "term_id": "GO:0030198",
  "gene_name": "A disintegrin and metalloproteinase with thrombospondin motifs 19",
  "gene": "UniProtKB:Q8TE59"
}